{
  "term_label": "exocytic vesicle",
  "term_id": "GO:0070382",
  "gene_symbol": "SYT3",
  "gene": "UniProtKB:Q9BQG1",
  "gene_name": "Synaptotagmin-3"
}